{
  "gene_symbol": "PPP4R4",
  "gene": "UniProtKB:Q6NUP7",
  "gene_name": "Serine_threonine-protein phosphatase 4 regulatory subunit 4",
  "term_label": "Unknown biological process",
  "term_id": "UNKNOWN:0002"
}